{
  "term_id": "GO:0048246",
  "gene": "UniProtKB:Q96LR4",
  "term_label": "macrophage chemotaxis",
  "gene_name": "Chemokine-like protein TAFA-4",
  "gene_symbol": "TAFA4"
}